{
  "term_label": "Unknown cellular component",
  "gene_symbol": "NPIPB2",
  "gene": "UniProtKB:A6NJ64",
  "term_id": "UNKNOWN:0003",
  "gene_name": "Putative nuclear pore complex-interacting protein family member B2"
}